{
  "term_label": "defense response to virus",
  "gene_symbol": "IFNL4",
  "term_id": "GO:0051607",
  "gene": "UniProtKB:K9M1U5",
  "gene_name": "Interferon lambda-4"
}